{
  "term_id": "GO:0008203",
  "gene_symbol": "CYP11A1",
  "gene_name": "Cholesterol side-chain cleavage enzyme, mitochondrial",
  "gene": "UniProtKB:P05108",
  "term_label": "cholesterol metabolic process"
}